regulation of intestinal lipid absorption [GO:1904729] (biological process) Definition: Any process that modulates the frequency, rate or extent of intestinal lipid absorption. Subtypes: regulation of intestinal cholesterol absorption [GO:0030300], negative regulation of intestinal lipid absorption [GO:1904730], positive regulation of intestinal lipid absorption [GO:1904731] Relationships: is a type of regulation of intestinal absorption [GO:1904478]; regulates intestinal lipid absorption [GO:0098856] References: PMID:18768481 Sources: GOC:TermGenie, GO_REF:0000058